hemoglobin binding [GO:0030492] (molecular function) Sources: GOC:jl Subtypes: hemoglobin alpha binding [GO:0031721], hemoglobin beta binding [GO:0031722] Relationships: is a type of protein binding [GO:0005515] Also known as: globin binding, haemoglobin binding Definition: Binding to hemoglobin, an oxygen carrying, conjugated protein containing four heme groups and globin.